{
  "term_label": "Unknown biological process",
  "gene_name": "Serine_threonine-protein phosphatase 2A 55 kDa regulatory subunit B alpha isoform",
  "term_id": "UNKNOWN:0002",
  "gene_symbol": "PPP2R2A",
  "gene": "UniProtKB:P63151"
}